{
  "term_label": "chemokine activity",
  "gene_name": "C-C motif chemokine 8",
  "gene": "UniProtKB:P80075",
  "gene_symbol": "CCL8",
  "term_id": "GO:0008009"
}